prospore septin ring [GO:0032169] (cellular component) Definition: A tight ring-shaped structure that forms in the division plane at the site of cytokinesis in a prospore; composed of septins as well as septin-associated proteins. References: PMID:16151244 Sources: GOC:krc, GOC:mah Relationships: is a type of GO:0005940; is a type of GO:0032161; is part of ascospore-type prospore [GO:0042764]